{
  "gene_symbol": "GTPBP2",
  "term_label": "translational elongation",
  "gene_name": "GTP-binding protein 2",
  "term_id": "GO:0006414",
  "gene": "UniProtKB:Q9BX10"
}